mitotic G2 DNA damage checkpoint signaling [GO:0007095] (biological process) Definition: A mitotic cell cycle checkpoint that detects and negatively regulates progression through the G2/M transition of the cell cycle in response to DNA damage. References: PMID:16299494 Sources: GOC:mtg_cell_cycle Also known as: G2/M transition DNA damage checkpoint, mitotic G2 DNA damage checkpoint, mitotic cell cycle G2/M transition DNA damage checkpoint, signal transduction involved in G2 DNA damage checkpoint, signal transduction involved in G2/M transition DNA damage checkpoint, signal transduction involved in mitotic G2 DNA damage checkpoint, signal transduction involved in mitotic G2/M transition DNA damage checkpoint, down regulation of signal transduction involved in mitotic G2 DNA damage checkpoint, down regulation of signal transduction involved in mitotic G2/M transition DNA damage checkpoint, down-regulation of signal transduction involved in mitotic G2 DNA damage checkpoint, down-regulation of signal transduction involved in mitotic G2/M transition DNA damage checkpoint, inhibition of signal transduction involved in mitotic G2 DNA damage checkpoint, negative regulation of signal transduction involved in mitotic G2 DNA damage checkpoint, negative regulation of signal transduction involved in mitotic G2/M transition DNA damage checkpoint, positive regulation of signal transduction involved in mitotic G2 DNA damage checkpoint, positive regulation of signal transduction involved in mitotic G2/M transition DNA damage checkpoint, regulation of signal transduction involved in mitotic G2 DNA damage checkpoint, regulation of signal transduction involved in mitotic G2/M transition DNA damage checkpoint, G2 DNA damage checkpoint Relationships: is a type of mitotic DNA damage checkpoint signaling [GO:0044773]; is a type of mitotic G2/M transition checkpoint [GO:0044818]; RO_0002092 mitotic G2 phase [GO:0000085]